regulation of systemic arterial blood pressure by circulatory renin-angiotensin [GO:0001991] (biological process) Relationships: is a type of GO:0003081 Definition: The process in which angiotensinogen metabolites in the bloodstream modulate the force with which blood passes through the circulatory system. The process begins when renin is released and cleaves angiotensinogen. Also known as: circulatory renin-angiotensin blood pressure regulation, circulatory renin-angiotensin regulation of blood pressure, circulatory renin-angiotensin control of blood pressure, control of blood pressure by circulatory renin-angiotensin, renin-angiotensin blood pressure control Sources: ISBN:0721643949